pantothenate catabolic process [GO:0015941] (biological process) Also known as: pantothenate breakdown, pantothenate catabolism, pantothenate degradation, vitamin B5 catabolic process, vitamin B5 catabolism Definition: The chemical reactions and pathways resulting in the breakdown of pantothenate, the anion of pantothenic acid. It is a B complex vitamin that is a constituent of coenzyme A and is distributed ubiquitously in foods. Sources: GOC:ai, ISBN:0721662544 Relationships: is a type of pantothenate metabolic process [GO:0015939]; is a type of modified amino acid catabolic process [GO:0042219]; is a type of water-soluble vitamin catabolic process [GO:0042365]; is a type of GO:0072329